{
  "gene": "UniProtKB:O75494",
  "gene_symbol": "SRSF10",
  "term_id": "GO:0000381",
  "term_label": "regulation of alternative mRNA splicing, via spliceosome",
  "gene_name": "Serine_arginine-rich splicing factor 10"
}